positive regulation of protein adenylylation [GO:1900724] (biological process) Definition: Any process that activates or increases the frequency, rate or extent of protein adenylylation. Sources: GOC:TermGenie Also known as: activation of protein AMPylation, activation of protein adenylation, activation of protein amino acid adenylylation, positive regulation of protein AMPylation, positive regulation of protein adenylation, positive regulation of protein amino acid adenylylation, up regulation of protein AMPylation, up regulation of protein adenylation, up regulation of protein adenylylation, up regulation of protein amino acid adenylylation, up-regulation of protein AMPylation, up-regulation of protein adenylation, up-regulation of protein adenylylation, up-regulation of protein amino acid adenylylation, upregulation of protein AMPylation, upregulation of protein adenylation, upregulation of protein adenylylation, upregulation of protein amino acid adenylylation, activation of protein adenylylation Relationships: is a type of positive regulation of protein modification process [GO:0031401]; is a type of GO:1900722; positively regulates GO:0018117